{
  "gene_symbol": "PATE1",
  "gene": "UniProtKB:Q8WXA2",
  "gene_name": "Prostate and testis expressed protein 1",
  "term_id": "UNKNOWN:0001",
  "term_label": "Unknown molecular function"
}